{
  "term_id": "UNKNOWN:0001",
  "gene": "UniProtKB:Q8N137",
  "term_label": "Unknown molecular function",
  "gene_name": "Centrobin",
  "gene_symbol": "CNTROB"
}